{
  "term_label": "Unknown cellular component",
  "gene_symbol": "PAMR1",
  "gene_name": "Inactive serine protease PAMR1",
  "gene": "UniProtKB:Q6UXH9",
  "term_id": "UNKNOWN:0003"
}